{
  "term_label": "Unknown biological process",
  "gene_symbol": "GMPR2",
  "gene_name": "GMP reductase 2",
  "term_id": "UNKNOWN:0002",
  "gene": "UniProtKB:Q9P2T1"
}